{
  "term_label": "Unknown cellular component",
  "term_id": "UNKNOWN:0003",
  "gene_name": "Uncharacterized protein C1orf122",
  "gene": "UniProtKB:Q6ZSJ8",
  "gene_symbol": "C1orf122"
}